{
  "gene": "UniProtKB:H3BV12",
  "gene_symbol": "GOLGA8Q",
  "term_id": "UNKNOWN:0001",
  "term_label": "Unknown molecular function",
  "gene_name": "Golgin subfamily A member 8Q"
}